{
  "gene_name": "Lipid droplet-regulating VLDL assembly factor AUP1",
  "term_id": "GO:0036503",
  "term_label": "ERAD pathway",
  "gene_symbol": "AUP1",
  "gene": "UniProtKB:Q9Y679"
}